cyclase inhibitor activity [GO:0010852] (molecular function) Subtypes: GO:0010855, guanylate cyclase inhibitor activity [GO:0030251] Sources: GOC:dph, GOC:tb Definition: Binds to and decreases the activity of an enzyme that catalyzes a ring closure reaction. Relationships: is a type of enzyme inhibitor activity [GO:0004857]; is a type of cyclase regulator activity [GO:0010851]; negatively regulates cyclase activity [GO:0009975]